positive regulation of protein localization to actin cortical patch [GO:1904372] (BP) Definition: Any process that activates or increases the frequency, rate or extent of protein localization to actin cortical patch. References: PMID:18216290 Sources: GOC:TermGenie, GO_REF:0000058 Also known as: positive regulation of protein localisation to actin cortical patch, up regulation of protein localisation to actin cortical patch, up regulation of protein localization to actin cortical patch, up-regulation of protein localisation to actin cortical patch, up-regulation of protein localization to actin cortical patch, upregulation of protein localisation to actin cortical patch, upregulation of protein localization to actin cortical patch, activation of protein localisation to actin cortical patch, activation of protein localization to actin cortical patch Relationships: is a type of regulation of protein localization to actin cortical patch [GO:1904370]; is a type of GO:1904778; positively regulates protein localization to actin cortical patch [GO:0044379]